N-terminal peptidyl-L-cysteine N-palmitoylation [GO:0018009] (biological process) Relationships: is a type of N-terminal protein palmitoylation [GO:0006500]; is_a peptidyl-cysteine modification [GO:0018198] Definition: The covalent attachment of a palmitoyl group to a nitrogen (N) atom in an N-terminal cysteine residue to form N-palmitoyl-L-cysteine. Sources: RESID:AA0060